{
  "term_label": "Unknown biological process",
  "term_id": "UNKNOWN:0002",
  "gene_symbol": "TRBJ1-3",
  "gene": "UniProtKB:A0A0J9YWP8",
  "gene_name": "T cell receptor beta joining 1-3"
}